{
  "gene_symbol": "ZNF280A",
  "gene": "UniProtKB:P59817",
  "gene_name": "Zinc finger protein 280A",
  "term_label": "DNA-binding transcription factor activity, RNA polymerase II-specific",
  "term_id": "GO:0000981"
}